{
  "term_id": "GO:0030674",
  "gene": "UniProtKB:Q9NZN4",
  "gene_symbol": "EHD2",
  "gene_name": "EH domain-containing protein 2",
  "term_label": "protein-macromolecule adaptor activity"
}